{
  "term_label": "Unknown biological process",
  "term_id": "UNKNOWN:0002",
  "gene": "UniProtKB:Q9Y2S2",
  "gene_name": "Lambda-crystallin homolog",
  "gene_symbol": "CRYL1"
}